{
  "gene": "UniProtKB:Q13428",
  "term_label": "nucleolus",
  "term_id": "GO:0005730",
  "gene_symbol": "TCOF1",
  "gene_name": "Treacle protein"
}